{
  "gene_name": "Receptor tyrosine-protein kinase erbB-4",
  "gene": "UniProtKB:Q15303",
  "term_label": "transmembrane receptor protein tyrosine kinase activity",
  "term_id": "GO:0004714",
  "gene_symbol": "ERBB4"
}